{
  "term_label": "clathrin adaptor activity",
  "gene": "UniProtKB:Q9Y6Q2",
  "gene_symbol": "STON1",
  "term_id": "GO:0035615",
  "gene_name": "Stonin-1"
}